plastid membrane organization [GO:0009668] (biological process) Also known as: plastid membrane organisation, plastid membrane organization and biogenesis Definition: A process that is carried out at the cellular level which results in the assembly, arrangement of constituent parts, or disassembly of either of the lipid bilayers surrounding a plastid. Relationships: is_a membrane organization [GO:0061024]; is part of plastid organization [GO:0009657] Sources: GOC:ai, GOC:dph, GOC:jl, GOC:mah Subtypes: plastid outer membrane organization [GO:0009666], GO:0009667, GO:0010027